{
  "term_label": "mitochondrial matrix",
  "gene": "UniProtKB:Q53S33",
  "gene_name": "BolA-like protein 3",
  "gene_symbol": "BOLA3",
  "term_id": "GO:0005759"
}